{
  "term_label": "Unknown biological process",
  "gene": "UniProtKB:Q68G75",
  "gene_symbol": "LEMD1",
  "term_id": "UNKNOWN:0002",
  "gene_name": "LEM domain-containing protein 1"
}